{
  "gene": "UniProtKB:Q8N9G6",
  "gene_symbol": "Q8N9G6",
  "gene_name": "Putative UPF0607 protein FLJ37424",
  "term_id": "UNKNOWN:0001",
  "term_label": "Unknown molecular function"
}